{
  "gene_symbol": "ACER2",
  "gene": "UniProtKB:Q5QJU3",
  "term_label": "N-acylsphingosine amidohydrolase activity",
  "term_id": "GO:0017040",
  "gene_name": "Alkaline ceramidase 2"
}